regulation of mitotic DNA replication initiation from early origin [GO:0062212] (biological process) Also known as: regulation of early replication origin firing Relationships: is a type of regulation of mitotic DNA replication initiation [GO:1903466] Definition: Any process that modulates the frequency, rate or extent of firing from an early origin of replication involved in mitotic DNA replication. References: PMID:22279046